{
  "term_label": "plasma membrane",
  "gene_name": "Sodium_hydrogen exchanger 2",
  "term_id": "GO:0005886",
  "gene_symbol": "SLC9A2",
  "gene": "UniProtKB:Q9UBY0"
}